{
  "term_label": "Unknown cellular component",
  "gene_name": "E3 ubiquitin-protein ligase TRIM41",
  "gene_symbol": "TRIM41",
  "term_id": "UNKNOWN:0003",
  "gene": "UniProtKB:Q8WV44"
}